negative regulation of multicellular organismal process [GO:0051241] (biological process) Sources: GOC:ai Definition: Any process that stops, prevents, or reduces the frequency, rate or extent of an organismal process, the processes pertinent to the function of an organism above the cellular level; includes the integrated processes of tissues and organs. Also known as: down regulation of multicellular organismal process, down-regulation of multicellular organismal process, downregulation of multicellular organismal process, inhibition of multicellular organismal process Subtypes: negative regulation of cytokine production [GO:0001818], negative regulation of tolerance induction [GO:0002644], GO:0003105, negative regulation of Wnt signaling pathway involved in heart development [GO:0003308], GO:0010633, GO:0010719, negative regulation of very-low-density lipoprotein particle remodeling [GO:0010903], negative regulation of lipoprotein particle clearance [GO:0010985], negative regulation of muscle hypertrophy [GO:0014741], negative regulation of muscle adaptation [GO:0014745], negative regulation of ossification [GO:0030279], GO:0031645, GO:0031651, negative regulation of heat dissipation [GO:0031655], negative regulation of gonadotropin secretion [GO:0032277], negative regulation of inhibin secretion [GO:0032339], GO:0032900, GO:0033600, negative regulation of tissue remodeling [GO:0034104], negative regulation of plasma lipoprotein oxidation [GO:0034445], negative regulation of terminal cell fate specification, open tracheal system [GO:0035155], negative regulation of fusion cell fate specification [GO:0035157], negative regulation of leukotriene production involved in inflammatory response [GO:0035492], GO:0035814, negative regulation of multicellular organism growth [GO:0040015], negative regulation of hair cycle [GO:0042636], negative regulation of fusion of sperm to egg plasma membrane [GO:0043013], negative regulation of keratinocyte differentiation [GO:0045617], negative regulation of embryo sac central cell differentiation [GO:0045692], GO:0045695, negative regulation of synergid differentiation [GO:0045698], negative regulation of spermatid nuclear differentiation [GO:0045701], negative regulation of salivary gland boundary specification [GO:0045705], negative regulation of chitin-based cuticle tanning [GO:0045800], GO:0045804, GO:0045906, negative regulation of muscle contraction [GO:0045932], negative regulation of juvenile hormone secretion [GO:0045972], negative regulation of embryonic development [GO:0045992], negative regulation of photoreceptor cell differentiation [GO:0046533], negative regulation of organ growth [GO:0046621], negative regulation of cuticle pigmentation [GO:0048080], negative regulation of female pigmentation [GO:0048090], GO:0048092, GO:0048521, negative regulation of post-embryonic development [GO:0048581], negative regulation of muscle organ development [GO:0048635], negative regulation of coagulation [GO:0050819], negative regulation of cell activation [GO:0050866], GO:0051460, negative regulation of hair follicle development [GO:0051799], negative regulation of nervous system development [GO:0051961], negative regulation of respiratory burst involved in inflammatory response [GO:0060266], negative regulation of ovulation [GO:0060280], negative regulation of penile erection [GO:0060407], negative regulation of digestive system process [GO:0060457], negative regulation of epithelial cell proliferation involved in prostate gland development [GO:0060770], GO:0061037, negative regulation of branching involved in lung morphogenesis [GO:0061048], negative regulation of cardiac endothelial to mesenchymal transition [GO:0062001], GO:0070164, negative regulation of mucus secretion [GO:0070256], GO:0070367, negative regulation of mesenchymal cell proliferation involved in ureter development [GO:0072200], negative regulation of spore-bearing organ development [GO:0075262], negative regulation of kidney development [GO:0090185], negative regulation of branching involved in ureteric bud morphogenesis [GO:0090191], GO:0110038, negative regulation of imaginal disc-derived wing vein specification [GO:0110109], negative regulation of animal organ morphogenesis [GO:0110111], negative regulation of cold-induced thermogenesis [GO:0120163], negative regulation of adenylate cyclase-activating adrenergic receptor signaling pathway involved in heart process [GO:0140199], negative regulation of transport across blood-brain barrier [GO:0150202], GO:1900033, negative regulation of amyloid-beta clearance [GO:1900222], GO:1901078, negative regulation of trophoblast cell migration [GO:1901164], negative regulation of lung ciliated cell differentiation [GO:1901247], negative regulation of lung goblet cell differentiation [GO:1901250], negative regulation of vasculature development [GO:1901343], negative regulation of seed dormancy process [GO:1902039], negative regulation of stem cell population maintenance [GO:1902455], negative regulation of sperm capacitation [GO:1902491], GO:1902747, negative regulation of renal amino acid absorption [GO:1902753], negative regulation of retina development in camera-type eye [GO:1902867], negative regulation of embryonic pattern specification [GO:1902876], negative regulation of bone development [GO:1903011], negative regulation of tube lumen cavitation [GO:1903133], negative regulation of vitellogenesis [GO:1903187], negative regulation of fear response [GO:1903366], negative regulation of renal phosphate excretion [GO:1903403], negative regulation of lactation [GO:1903488], GO:1903523, negative regulation of epithelial cell-cell adhesion involved in epithelium migration [GO:1903682], negative regulation of hemopoiesis [GO:1903707], GO:1903815, GO:1903941, negative regulation of adipose tissue development [GO:1904178], negative regulation of transcytosis [GO:1904299], GO:1904302, negative regulation of cardiac ventricle development [GO:1904413], negative regulation of thyroid gland epithelial cell proliferation [GO:1904442], negative regulation of lung alveolus development [GO:1904654], GO:1904839, negative regulation of apical ectodermal ridge formation [GO:1905141], negative regulation of cardiocyte differentiation [GO:1905208], GO:1905277, negative regulation of epidermal growth factor receptor signaling pathway involved in heart process [GO:1905283], GO:1905293, GO:1905299, negative regulation of plant organ morphogenesis [GO:1905422], GO:1905622, negative regulation of oogenesis [GO:1905880], negative regulation of germ cell proliferation [GO:1905937], negative regulation of gonad development [GO:1905940], negative regulation of endothelial tube morphogenesis [GO:1905955], negative regulation of determination of dorsal identity [GO:2000016], negative regulation of ureter smooth muscle cell differentiation [GO:2000062], negative regulation of type B pancreatic cell development [GO:2000077], negative regulation of mammary stem cell proliferation [GO:2000102], negative regulation of branching morphogenesis of a nerve [GO:2000173], negative regulation of pancreatic A cell differentiation [GO:2000227], negative regulation of renal albumin absorption [GO:2000533], negative regulation of seed maturation [GO:2000692], GO:2000791, negative regulation of parathyroid hormone secretion [GO:2000829], negative regulation of steroid hormone secretion [GO:2000832], negative regulation of lens epithelial cell proliferation [GO:2001110], negative regulation of renal water transport [GO:2001152] Relationships: is_a GO:0048519; is a type of regulation of multicellular organismal process [GO:0051239]; negatively regulates multicellular organismal process [GO:0032501]